{
  "term_label": "chemorepellent activity",
  "gene_symbol": "SEMA6A",
  "term_id": "GO:0045499",
  "gene": "UniProtKB:Q9H2E6",
  "gene_name": "Semaphorin-6A"
}